{
  "gene": "UniProtKB:Q9ULB5",
  "term_label": "catenin complex",
  "gene_symbol": "CDH7",
  "term_id": "GO:0016342",
  "gene_name": "Cadherin-7"
}